{
  "gene": "UniProtKB:Q3KNW1",
  "gene_name": "Zinc finger protein SNAI3",
  "term_label": "regulation of DNA-templated transcription",
  "gene_symbol": "SNAI3",
  "term_id": "GO:0006355"
}